{
  "gene_symbol": "RNF126",
  "gene": "UniProtKB:Q9BV68",
  "term_id": "GO:0016567",
  "gene_name": "E3 ubiquitin-protein ligase RNF126",
  "term_label": "protein ubiquitination"
}